{
  "gene_symbol": "THAP9",
  "gene_name": "DNA transposase THAP9",
  "term_label": "DNA binding",
  "term_id": "GO:0003677",
  "gene": "UniProtKB:Q9H5L6"
}